{
  "gene_name": "Ubiquitin carboxyl-terminal hydrolase 6",
  "gene": "UniProtKB:P35125",
  "gene_symbol": "USP6",
  "term_label": "Golgi apparatus",
  "term_id": "GO:0005794"
}